{
  "term_id": "GO:0005886",
  "term_label": "plasma membrane",
  "gene_symbol": "TSPAN8",
  "gene_name": "Tetraspanin-8",
  "gene": "UniProtKB:P19075"
}